{
  "gene": "UniProtKB:A0A075B6T6",
  "gene_symbol": "TRAV12-2",
  "term_label": "peptide antigen binding",
  "term_id": "GO:0042605",
  "gene_name": "T cell receptor alpha variable 12-2"
}